(R)-2-hydroxyglutarate-pyruvate transhydrogenase activity [GO:0099615] (molecular function) Also known as: (D)-2-hydroxyglutarate-pyruvate transhydrogenase activity, D-2HG-pyruvate transhydrogenase activity, R-2-hydroxyglutarate alpha-pyruvate transhydrogenase activity Definition: Catalysis of the reaction: (R)-2-hydroxyglutarate + pyruvate = (R)-lactate + 2-oxoglutarate. Relationships: is a type of (R)-2-hydroxyglutarate dehydrogenase activity [GO:0051990] References: PMID:26774271 Sources: RHEA:51608